{
  "gene": "UniProtKB:Q5MJ08",
  "gene_symbol": "SPANXN4",
  "gene_name": "Sperm protein associated with the nucleus on the X chromosome N4",
  "term_label": "Unknown molecular function",
  "term_id": "UNKNOWN:0001"
}